positive regulation of production of molecular mediator of immune response [GO:0002702] (biological process) Subtypes: positive regulation of antimicrobial peptide production [GO:0002225], positive regulation of immunoglobulin production [GO:0002639], positive regulation of cytokine production involved in immune response [GO:0002720], GO:0071663, GO:2000513 Definition: Any process that activates or increases the frequency, rate, or extent of the production of molecular mediator of immune response. Relationships: is a type of positive regulation of immune effector process [GO:0002699]; is_a regulation of production of molecular mediator of immune response [GO:0002700]; is a type of positive regulation of gene expression [GO:0010628]; positively regulates production of molecular mediator of immune response [GO:0002440] Also known as: up regulation of production of molecular mediator of immune response, up-regulation of production of molecular mediator of immune response, upregulation of production of molecular mediator of immune response, activation of production of molecular mediator of immune response, stimulation of production of molecular mediator of immune response Sources: GOC:add